{
  "term_label": "extracellular space",
  "term_id": "GO:0005615",
  "gene_name": "WAP four-disulfide core domain protein 10A",
  "gene_symbol": "WFDC10A",
  "gene": "UniProtKB:Q9H1F0"
}